{
  "term_label": "nucleus",
  "gene": "UniProtKB:Q8N9U0",
  "gene_name": "Tandem C2 domains nuclear protein",
  "term_id": "GO:0005634",
  "gene_symbol": "TC2N"
}